{
  "gene_symbol": "GPR61",
  "gene_name": "G-protein coupled receptor 61",
  "gene": "UniProtKB:Q9BZJ8",
  "term_id": "GO:0038035",
  "term_label": "ligand-independent adenylate cyclase-activating G protein-coupled receptor signaling pathway"
}